{
  "term_label": "Unknown biological process",
  "gene_symbol": "SIL1",
  "gene_name": "Nucleotide exchange factor SIL1",
  "gene": "UniProtKB:Q9H173",
  "term_id": "UNKNOWN:0002"
}